{
  "term_label": "glutathione metabolic process",
  "term_id": "GO:0006749",
  "gene_name": "Glutathione S-transferase theta-4",
  "gene_symbol": "GSTT4",
  "gene": "UniProtKB:A0A1W2PR19"
}